{
  "term_label": "GDP phosphatase activity",
  "gene": "UniProtKB:Q8WVQ1",
  "gene_symbol": "CANT1",
  "gene_name": "Soluble calcium-activated nucleotidase 1",
  "term_id": "GO:0004382"
}